{
  "gene_symbol": "CMC1",
  "term_label": "Unknown molecular function",
  "gene_name": "COX assembly mitochondrial protein homolog",
  "term_id": "UNKNOWN:0001",
  "gene": "UniProtKB:Q7Z7K0"
}